{
  "term_id": "GO:0030335",
  "gene": "UniProtKB:Q9NS98",
  "term_label": "positive regulation of cell migration",
  "gene_name": "Semaphorin-3G",
  "gene_symbol": "SEMA3G"
}